adenine binding [GO:0002055] (molecular function) Also known as: 6-aminopurine binding Sources: GOC:hjd Definition: Binding to adenine, a purine base. Relationships: is a type of purine nucleobase binding [GO:0002060]